{
  "gene_symbol": "MYLK",
  "gene_name": "Myosin light chain kinase, smooth muscle",
  "term_label": "stress fiber",
  "gene": "UniProtKB:Q15746",
  "term_id": "GO:0001725"
}